regulation of palmitic acid catabolic process [GO:0106393] (biological process) Definition: Any process that modulates the frequency, rate or extent of a palmitic acid catabolic process. Subtypes: negative regulation of palmitic acid catabolic process [GO:0106394], positive regulation of palmitic acid catabolic process [GO:0106395] References: PMID:14677856 Relationships: is a type of regulation of fatty acid metabolic process [GO:0019217]; is a type of regulation of lipid catabolic process [GO:0050994]; regulates palmitic acid catabolic process [GO:1900534]